{
  "term_label": "plasma membrane",
  "gene_symbol": "PCDHB8",
  "gene_name": "Protocadherin beta-8",
  "gene": "UniProtKB:Q9UN66",
  "term_id": "GO:0005886"
}